right ventral basal body [GO:1902676] (cellular component) References: PMID:16607022, PMID:5961344 Sources: GOC:TermGenie, GOC:giardia, GO_REF:0000064, ISBN:9780124260207 Definition: Any ciliary basal body that is part of a right ventral flagellum found in Giardia species (trophozoite stage). Relationships: is a type of ciliary basal body [GO:0036064]; is part of right ventral flagellum [GO:0097559] Note: Note that we deem cilium and microtubule-based flagellum to be equivalent. Also note that, due to the asymmetric nature of the Giardia trophozoite, this term is defined spatially as the trophozoite is viewed from the dorsal side, with the two nuclei dorsal to the ventral disc, and the ventral disc toward the anterior. Also known as: cilial basal body of right ventral cilium, cilial basal body of right ventral flagellum, ciliary basal body of right ventral cilium, ciliary basal body of right ventral flagellum, cilium basal body of right ventral cilium, cilium basal body of right ventral flagellum, microtubule basal body of right ventral cilium, microtubule basal body of right ventral flagellum, right ventral flagellum ciliary basal body